{
  "gene": "UniProtKB:P41250",
  "gene_symbol": "GARS1",
  "term_id": "GO:0070150",
  "gene_name": "Glycine--tRNA ligase",
  "term_label": "mitochondrial glycyl-tRNA aminoacylation"
}